fructose transmembrane transport [GO:0015755] (biological process) Subtypes: fructose export from vacuole to cytoplasm [GO:1902334], fructose import across plasma membrane [GO:1990539] Definition: The directed movement of fructose into, out of or within a cell, or between cells, by means of some agent such as a transporter or pore. Fructose exists in a open chain form or as a ring compound. D-fructose is the sweetest of the sugars and is found free in a large number of fruits and honey. Sources: GOC:ai Also known as: fructose transport Relationships: is a type of hexose transmembrane transport [GO:0008645]